mitotic actomyosin contractile ring contraction [GO:1902404] (biological process) Definition: Any actomyosin contractile ring contraction that is involved in mitotic cell cycle. Regulation: RO_0002211 by GO:1903471; negatively regulated by negative regulation of mitotic actomyosin contractile ring contraction [GO:1903472]; positively regulated by positive regulation of mitotic actomyosin contractile ring contraction [GO:1903473] Sources: GOC:TermGenie, GOC:mtg_cell_cycle Also known as: contractile ring contraction involved in cell cycle cytokinesis involved in mitotic cell cycle, cytokinesis, actomyosin ring contraction involved in mitotic cell cycle, mitotic actomyosin contractile ring constriction Relationships: is a type of GO:0000916; is a type of mitotic cytokinetic process [GO:1902410]